{
  "term_label": "Golgi cisterna",
  "term_id": "GO:0031985",
  "gene_symbol": "RAB30",
  "gene_name": "Ras-related protein Rab-30",
  "gene": "UniProtKB:Q15771"
}